{
  "gene": "UniProtKB:A0A2R8YEV3",
  "gene_name": "Olfactory receptor",
  "term_label": "Unknown cellular component",
  "gene_symbol": "OR2A42",
  "term_id": "UNKNOWN:0003"
}